{
  "gene_symbol": "PSMG2",
  "gene": "UniProtKB:Q969U7",
  "term_id": "GO:0060090",
  "term_label": "molecular adaptor activity",
  "gene_name": "Proteasome assembly chaperone 2"
}